{
  "gene_name": "HLA class II histocompatibility antigen, DO beta chain",
  "term_id": "GO:0023026",
  "gene": "UniProtKB:P13765",
  "term_label": "MHC class II protein complex binding",
  "gene_symbol": "HLA-DOB"
}